negative regulation of neurofibrillary tangle assembly [GO:1902997] (biological process) Relationships: is_a negative regulation of inclusion body assembly [GO:0090084]; is a type of regulation of neurofibrillary tangle assembly [GO:1902996]; negatively regulates neurofibrillary tangle assembly [GO:1902988] Also known as: down regulation of neurofibrillary tangle assembly, down regulation of neurofibrillary tangle formation, down-regulation of neurofibrillary tangle assembly, down-regulation of neurofibrillary tangle formation, downregulation of neurofibrillary tangle assembly, downregulation of neurofibrillary tangle formation, negative regulation of neurofibrillary tangle formation, down regulation of flame-shaped neurofibrillary tangle assembly, down regulation of flame-shaped neurofibrillary tangle formation, down regulation of star-shaped neurofibrillary tangle assembly, down regulation of star-shaped neurofibrillary tangle formation, down-regulation of flame-shaped neurofibrillary tangle assembly, down-regulation of flame-shaped neurofibrillary tangle formation, down-regulation of star-shaped neurofibrillary tangle assembly, down-regulation of star-shaped neurofibrillary tangle formation, downregulation of flame-shaped neurofibrillary tangle assembly, downregulation of flame-shaped neurofibrillary tangle formation, downregulation of star-shaped neurofibrillary tangle assembly, downregulation of star-shaped neurofibrillary tangle formation, inhibition of flame-shaped neurofibrillary tangle assembly, inhibition of flame-shaped neurofibrillary tangle formation, inhibition of neurofibrillary tangle assembly, inhibition of neurofibrillary tangle formation, inhibition of star-shaped neurofibrillary tangle assembly, inhibition of star-shaped neurofibrillary tangle formation, negative regulation of flame-shaped neurofibrillary tangle assembly, negative regulation of flame-shaped neurofibrillary tangle formation, negative regulation of star-shaped neurofibrillary tangle assembly, negative regulation of star-shaped neurofibrillary tangle formation Definition: Any process that stops, prevents or reduces the frequency, rate or extent of neurofibrillary tangle assembly. References: PMID:15897157 Sources: GOC:TermGenie, GOC:sjp, GO_REF:0000058